{
  "gene": "UniProtKB:O60890",
  "gene_symbol": "OPHN1",
  "gene_name": "Oligophrenin-1",
  "term_id": "GO:0015629",
  "term_label": "actin cytoskeleton"
}